{
  "gene": "UniProtKB:P11388",
  "gene_symbol": "TOP2A",
  "gene_name": "DNA topoisomerase 2-alpha",
  "term_label": "sister chromatid segregation",
  "term_id": "GO:0000819"
}